{
  "term_id": "GO:0034446",
  "term_label": "substrate adhesion-dependent cell spreading",
  "gene_name": "Laminin subunit beta-3",
  "gene": "UniProtKB:Q13751",
  "gene_symbol": "LAMB3"
}